stress response to cadmium ion [GO:1990170] (biological process) Also known as: stress response to cadmium, response to cadmium ion stress, response to cadmium toxicity Relationships: is_a response to cadmium ion [GO:0046686]; is a type of GO:0097501 Definition: Any process that results in a change in state or activity of a cell or an organism (in terms of movement, secretion, enzyme production, gene expression, etc.) as a result of a disturbance in organismal or cellular homeostasis caused by a cadmium ion stimulus. Sources: GOC:kmv